{
  "gene_symbol": "SKOR2",
  "gene": "UniProtKB:Q2VWA4",
  "term_label": "negative regulation of transcription by RNA polymerase II",
  "term_id": "GO:0000122",
  "gene_name": "SKI family transcriptional corepressor 2"
}